{
  "gene_name": "PDZ and LIM domain protein 5",
  "term_id": "GO:0005912",
  "gene": "UniProtKB:Q96HC4",
  "gene_symbol": "PDLIM5",
  "term_label": "adherens junction"
}